{
  "gene_symbol": "GRK3",
  "gene": "UniProtKB:P35626",
  "gene_name": "Beta-adrenergic receptor kinase 2",
  "term_label": "Unknown cellular component",
  "term_id": "UNKNOWN:0003"
}